{
  "term_id": "UNKNOWN:0002",
  "gene_symbol": "SAMD13",
  "gene": "UniProtKB:Q5VXD3",
  "term_label": "Unknown biological process",
  "gene_name": "Sterile alpha motif domain-containing protein 13"
}